{
  "gene_symbol": "ODF3L2",
  "gene": "UniProtKB:Q3SX64",
  "term_label": "Unknown biological process",
  "term_id": "UNKNOWN:0002",
  "gene_name": "Outer dense fiber protein 3-like protein 2"
}